{
  "gene": "UniProtKB:P46095",
  "term_label": "sphingosine-1-phosphate receptor activity",
  "term_id": "GO:0038036",
  "gene_name": "G-protein coupled receptor 6",
  "gene_symbol": "GPR6"
}